{
  "gene_name": "Histone-lysine N-methyltransferase EZH1",
  "gene": "UniProtKB:Q92800",
  "term_id": "GO:0031507",
  "term_label": "heterochromatin formation",
  "gene_symbol": "EZH1"
}